aliphatic amine oxidase activity [GO:0052595] (molecular function) Also known as: aliphatic-amine oxidase activity, aliphatic-amine:oxygen oxidoreductase(deaminating) activity Definition: Catalysis of the reaction: an aliphatic amine + H2O + O2 = an aldehyde + NH3 + hydrogen peroxide + H+. Subtypes: glycine oxidase activity [GO:0043799], ethanolamine oxidase activity [GO:0047883] Sources: MetaCyc:AMINEOXID-RXN Relationships: is a type of oxidoreductase activity, acting on the CH-NH2 group of donors, oxygen as acceptor [GO:0016641]; is_a GO:0030058